adrenal gland development [GO:0030325] (biological process) Relationships: is_a gland development [GO:0048732]; BFO_0000050 endocrine system development [GO:0035270] Also known as: interrenal gland Sources: GOC:dgh Definition: The process whose specific outcome is the progression of the adrenal gland over time, from its formation to the mature structure. This gland can either be a discrete structure located bilaterally above each kidney, or a cluster of cells in the head kidney that perform the functions of the adrenal gland. In either case, this organ consists of two cells types, aminergic chromaffin cells and steroidogenic cortical cells.